{
  "gene": "UniProtKB:Q8WVH0",
  "term_label": "modulation of chemical synaptic transmission",
  "gene_name": "Complexin-3",
  "gene_symbol": "CPLX3",
  "term_id": "GO:0050804"
}